guanosine tetraphosphate catabolic process [GO:0015971] (BP) Relationships: is a type of GO:0009154; is a type of guanosine tetraphosphate metabolic process [GO:0015969]; is a type of purine ribonucleoside bisphosphate catabolic process [GO:0034037] Also known as: guanosine tetraphosphate (5'-ppGpp-3') catabolic process, guanosine tetraphosphate (5'-ppGpp-3') catabolism, guanosine tetraphosphate breakdown, guanosine tetraphosphate catabolism, guanosine tetraphosphate degradation Sources: GOC:ai Definition: The chemical reactions and pathways resulting in the breakdown of guanine tetraphosphate (5'-ppGpp-3'), a derivative of guanine riboside with four phosphates.